{
  "gene_symbol": "ZFP3",
  "term_label": "nucleus",
  "gene": "UniProtKB:Q96NJ6",
  "gene_name": "Zinc finger protein 3 homolog",
  "term_id": "GO:0005634"
}